{
  "gene_symbol": "SLC35B2",
  "term_id": "GO:0055085",
  "gene": "UniProtKB:Q8TB61",
  "term_label": "transmembrane transport",
  "gene_name": "Adenosine 3'-phospho 5'-phosphosulfate transporter 1"
}